{
  "gene": "UniProtKB:Q70IA6",
  "gene_symbol": "MOB2",
  "term_id": "GO:0005737",
  "term_label": "cytoplasm",
  "gene_name": "MOB kinase activator 2"
}